{
  "gene": "UniProtKB:A0A0A6YYJ7",
  "term_label": "immunoglobulin complex",
  "gene_symbol": "TRAV8-3",
  "term_id": "GO:0019814",
  "gene_name": "T cell receptor alpha variable 8-3"
}